{
  "term_label": "Unknown cellular component",
  "term_id": "UNKNOWN:0003",
  "gene_symbol": "C19orf53",
  "gene_name": "Leydig cell tumor 10 kDa protein homolog",
  "gene": "UniProtKB:Q9UNZ5"
}